{
  "gene": "UniProtKB:O43555",
  "gene_symbol": "GNRH2",
  "term_label": "extracellular space",
  "gene_name": "Progonadoliberin-2",
  "term_id": "GO:0005615"
}